{
  "term_label": "negative regulation of transcription by RNA polymerase II",
  "gene_symbol": "SOX8",
  "term_id": "GO:0000122",
  "gene_name": "Transcription factor SOX-8",
  "gene": "UniProtKB:P57073"
}